{
  "term_label": "cytoplasm",
  "gene_name": "Ubiquitin-associated protein 2-like",
  "term_id": "GO:0005737",
  "gene": "UniProtKB:Q14157",
  "gene_symbol": "UBAP2L"
}